{
  "gene_name": "Haloacid dehalogenase-like hydrolase domain-containing protein 2",
  "gene": "UniProtKB:Q9H0R4",
  "gene_symbol": "HDHD2",
  "term_id": "UNKNOWN:0002",
  "term_label": "Unknown biological process"
}